{
  "gene_name": "Twinfilin-2",
  "gene": "UniProtKB:Q6IBS0",
  "term_id": "GO:0030016",
  "gene_symbol": "TWF2",
  "term_label": "myofibril"
}